oxidoreductase activity, acting on the CH-NH group of donors, oxygen as acceptor [GO:0016647] (molecular function) Relationships: is a type of oxidoreductase activity, acting on the CH-NH group of donors [GO:0016645] Subtypes: dihydropterin oxidase activity [GO:0004154], GO:0008115, hydroxy-nicotine oxidase activity [GO:0019116], polyamine oxidase activity [GO:0046592], dihydrobenzophenanthridine oxidase activity [GO:0047132], dimethylglycine oxidase activity [GO:0047866], L-pipecolate oxidase activity [GO:0050031], N-methyl-L-amino-acid oxidase activity [GO:0050131], N6-methyl-lysine oxidase activity [GO:0050134], GO:0051698, GO:0051700, coenzyme F420H2 oxidase activity [GO:0052765], 4-methylaminobutyrate oxidase (demethylating) activity [GO:0102317] Definition: Catalysis of an oxidation-reduction (redox) reaction in which a CH-NH group acts as a hydrogen or electron donor and reduces oxygen. Sources: GOC:jl